anterior semicircular canal development [GO:0060873] (biological process) Definition: The progession of the anterior semicircular canal from its initial formation to the mature structure. Relationships: is a type of semicircular canal development [GO:0060872] Sources: GOC:dph, GOC:sdb_2009, GOC:tb